{
  "term_id": "GO:0007218",
  "gene_symbol": "SSTR3",
  "gene": "UniProtKB:P32745",
  "gene_name": "Somatostatin receptor type 3",
  "term_label": "neuropeptide signaling pathway"
}